regulation of translation at presynapse, modulating synaptic transmission [GO:0099577] (biological process) Note: Note that this term was created for the SynGO project, and will be obsoleted when the SynGO annotations are made in Noctua. Relationships: is a type of presynaptic modulation of chemical synaptic transmission [GO:0099171]; is a type of regulation of translation at synapse, modulating synaptic transmission [GO:0099547]; is a type of regulation of translation at presynapse [GO:0140244] Definition: Any process that modulates synaptic transmission by regulating translation occurring at the presynapse. Sources: GOC:dos